{
  "term_id": "GO:0005886",
  "gene_name": "Anthrax toxin receptor 2",
  "term_label": "plasma membrane",
  "gene": "UniProtKB:P58335",
  "gene_symbol": "ANTXR2"
}